{
  "gene_name": "Protein FAM193B",
  "term_label": "nucleus",
  "term_id": "GO:0005634",
  "gene_symbol": "FAM193B",
  "gene": "UniProtKB:Q96PV7"
}